{
  "gene_symbol": "TCF21",
  "gene_name": "Transcription factor 21",
  "gene": "UniProtKB:O43680",
  "term_label": "RNA polymerase II transcription regulatory region sequence-specific DNA binding",
  "term_id": "GO:0000977"
}